pigment cell development [GO:0070285] (biological process) Relationships: is a type of cell development [GO:0048468]; is part of pigment cell differentiation [GO:0050931] Sources: GOC:cvs Definition: The process whose specific outcome is the progression of a pigment cell over time, from its formation to the mature structure. Cell development does not include the steps involved in committing a cell to a pigment cell fate.